{
  "gene_symbol": "DNM1L",
  "gene": "UniProtKB:O00429",
  "term_id": "GO:0016020",
  "gene_name": "Dynamin-1-like protein",
  "term_label": "membrane"
}